stress-induced homeostatically regulated protein degradation pathway [GO:0120174] (BP) Relationships: is a type of GO:0033554; is a type of proteasome-mediated ubiquitin-dependent protein catabolic process [GO:0043161]; is a type of response to nitrogen compound [GO:1901698] References: PMID:29861160 Sources: GOC:rl, GOC:rn Definition: A stress-inducible protein catabolic pathway that promotes protein quality control by accelerating the degradation of misfolded ER membrane and cytosolic proteins, as well as native proteins. The pathway starts with the activation, by stress, of the Nma111p/Ynm3p serine protease, which cleaves the stress-induced hydrophilin Roq1p, resulting in the generation of a Roq1p cleavage product that selectively interacts with Ubr1p, an E3 ubiquitin ligase. Interaction with the Ubr1p type-1 substrate binding site reprograms the substrate specificity of this ubiquitin ligase resulting in the selective proteasome-mediated degradation of misfolded and native proteins. The pathway ends with degradation of the protein by the cytoplasmic proteasome. Currently, NMA111, ROQ1, UBR1, RAD6, and CDC48 are considered to be involved in this quality control pathway. Note: Note, although the SHRED pathway may contain some components in common with ER-associated protein degradation (ERAD) pathways (GO:0036503), such as UBR1, RAD6 and CDC48, other ERAD components, such as HRD1 and DOA10 do not appear to be involved, and as such these pathways are currently considered to be distinct. ERAD pathways target misfolded ER lumenal proteins (ERAD-L), ER membrane proteins (ERAD-M) and ER proteins with misfolded cytosolic domains (ERAD-C) by recognizing aberrant proteins, retrotranslocating these substrates to the cytosol, followed by subsequent substrate ubiquitination and proteosome-mediated degradation. In contrast the SHRED pathway, although inducible by stress, targets diverse ER membrane and cytosolic proteins as well as numerous other native proteins in the absence of stress. In the SHRED pathway an Nma111p serine protease-mediated cleavage results in the generation of a Roq1p fragment that then binds to the type-1 active site of Ubr1p, altering its substrate specificity, and leading to the proteasome-mediated degradation of both misfolded and native proteins. SHRED is also considered to be distinct from the endoplasmic reticulum unfolded protein response (GO:0030968), a process by which ER stress activates the ER membrane protein Ire1p, resulting in splicing of the HAC1 mRNA, followed by Hac1p-mediated up-regulation of UPR genes. Induction of SHRED does not require IRE1 or HAC1, and as such is currently considered to be distinct. Also known as: SHRED pathway